positive regulation of isopentenyl diphosphate biosynthetic process, mevalonate pathway [GO:1900486] (BP) Relationships: is_a positive regulation of amide metabolic process [GO:0034250]; is a type of positive regulation of small molecule metabolic process [GO:0062013]; is a type of positive regulation of phospholipid biosynthetic process [GO:0071073]; is a type of regulation of isopentenyl diphosphate biosynthetic process, mevalonate pathway [GO:2001210]; positively regulates isoprenoid metabolic process [GO:0006720]; positively regulates isopentenyl diphosphate biosynthetic process, mevalonate pathway [GO:0019287] Sources: GOC:TermGenie Also known as: activation of Ac-MVA pathway, activation of acetate-mevalonate pathway, activation of isopentenyl diphosphate anabolism, mevalonate pathway, activation of isopentenyl diphosphate formation, mevalonate pathway, activation of isopentenyl diphosphate synthesis, mevalonate pathway, positive regulation of Ac-MVA pathway, positive regulation of acetate-mevalonate pathway, positive regulation of isopentenyl diphosphate anabolism, mevalonate pathway, positive regulation of isopentenyl diphosphate formation, mevalonate pathway, positive regulation of isopentenyl diphosphate synthesis, mevalonate pathway, up regulation of Ac-MVA pathway, up regulation of acetate-mevalonate pathway, up regulation of isopentenyl diphosphate anabolism, mevalonate pathway, up regulation of isopentenyl diphosphate biosynthetic process, mevalonate pathway, up regulation of isopentenyl diphosphate formation, mevalonate pathway, up regulation of isopentenyl diphosphate synthesis, mevalonate pathway, up-regulation of Ac-MVA pathway, up-regulation of acetate-mevalonate pathway, up-regulation of isopentenyl diphosphate anabolism, mevalonate pathway, up-regulation of isopentenyl diphosphate biosynthetic process, mevalonate pathway, up-regulation of isopentenyl diphosphate formation, mevalonate pathway, up-regulation of isopentenyl diphosphate synthesis, mevalonate pathway, upregulation of Ac-MVA pathway, upregulation of acetate-mevalonate pathway, upregulation of isopentenyl diphosphate anabolism, mevalonate pathway, upregulation of isopentenyl diphosphate biosynthetic process, mevalonate pathway, upregulation of isopentenyl diphosphate formation, mevalonate pathway, upregulation of isopentenyl diphosphate synthesis, mevalonate pathway, activation of isopentenyl diphosphate biosynthetic process, mevalonate pathway Definition: Any process that activates or increases the frequency, rate or extent of isopentenyl diphosphate biosynthetic process, mevalonate pathway.